regulation of oxidative phosphorylation [GO:0002082] (biological process) Sources: GOC:dph Definition: Any process that modulates the frequency, rate or extent of the chemical reactions and pathways resulting in the phosphorylation of ADP to ATP that accompanies the oxidation of a metabolite through the operation of the respiratory chain. Oxidation of compounds establishes a proton gradient across the membrane, providing the energy for ATP synthesis. Relationships: is a type of regulation of aerobic respiration [GO:1903715]; regulates oxidative phosphorylation [GO:0006119] Also known as: OXPHOS Subtypes: negative regulation of oxidative phosphorylation [GO:0090324], positive regulation of oxidative phosphorylation [GO:1903862]